response to ozone [GO:0010193] (biological process) Definition: Any process that results in a change in state or activity of a cell or an organism (in terms of movement, secretion, enzyme production, gene expression, etc.) as a result of a ozone stimulus. Subtypes: cellular response to ozone [GO:0071457] Relationships: is a type of GO:0000302 Sources: GOC:sm